{
  "gene": "UniProtKB:Q9H3M9",
  "term_label": "protein quality control for misfolded or incompletely synthesized proteins",
  "gene_symbol": "ATXN3L",
  "gene_name": "Ataxin-3-like protein",
  "term_id": "GO:0006515"
}